{
  "gene_name": "Signal peptidase complex catalytic subunit SEC11A",
  "gene": "UniProtKB:P67812",
  "gene_symbol": "SEC11A",
  "term_label": "peptidase activity",
  "term_id": "GO:0008233"
}